{
  "gene_name": "Putative coiled-coil domain-containing protein 196",
  "gene_symbol": "CCDC196",
  "term_label": "Unknown molecular function",
  "gene": "UniProtKB:A0A1B0GTZ2",
  "term_id": "UNKNOWN:0001"
}